thymine biosynthetic process [GO:0046106] (biological process) Relationships: is a type of GO:0019856; is a type of thymine metabolic process [GO:0019859] Also known as: thymine anabolism, thymine biosynthesis, thymine formation, thymine synthesis Definition: The chemical reactions and pathways resulting in the formation of thymine, 5-methyluracil, one of the two major pyrimidine bases present (as thymidine) in DNA but not found in RNA other than (as ribothymidine) in transfer RNA, where it is a minor base. Sources: GOC:go_curators